ATP-dependent activity, acting on RNA [GO:0008186] (molecular function) Definition: Catalysis of the reaction: ATP + H2O = ADP + phosphate; this reaction requires the presence of RNA, and it drives another reaction. Relationships: is a type of ATP-dependent activity [GO:0140657] Sources: GOC:jl Subtypes: RNA helicase activity [GO:0003724], DNA/RNA helicase activity [GO:0033677], RNA translocase activity [GO:0039630] Also known as: ATPase activity, acting on RNA, ATPase, acting on RNA, RNA-dependent ATPase activity, RNA-dependent adenosinetriphosphatase activity